positive regulation of septum digestion after cytokinesis [GO:2001043] (biological process) Sources: GOC:mtg_cell_cycle, GOC:obol Definition: Any process that activates or increases the frequency, rate or extent of the process of physically separating the septal cell wall material by enzymatic digestion, that occurs after daughter cells are separated by cytokinesis. Relationships: is a type of regulation of septum digestion after cytokinesis [GO:0010590]; is a type of positive regulation of cellular process [GO:0048522]; positively regulates septum digestion after cytokinesis [GO:0000920] Also known as: positive regulation of cell separation after cytokinesis, positive regulation of cytokinetic cell separation